{
  "gene": "UniProtKB:Q6PF04",
  "term_label": "regulation of transcription by RNA polymerase II",
  "gene_symbol": "ZNF613",
  "gene_name": "Zinc finger protein 613",
  "term_id": "GO:0006357"
}